{
  "gene_symbol": "TWF2",
  "term_label": "actin filament binding",
  "term_id": "GO:0051015",
  "gene": "UniProtKB:Q6IBS0",
  "gene_name": "Twinfilin-2"
}